{
  "term_id": "GO:0000978",
  "gene_symbol": "HES7",
  "gene": "UniProtKB:Q9BYE0",
  "term_label": "RNA polymerase II cis-regulatory region sequence-specific DNA binding",
  "gene_name": "Transcription factor HES-7"
}